{
  "gene_symbol": "ELF5",
  "gene_name": "ETS-related transcription factor Elf-5",
  "term_label": "cell differentiation",
  "term_id": "GO:0030154",
  "gene": "UniProtKB:Q9UKW6"
}